{
  "gene_symbol": "DRD3",
  "term_id": "GO:0060158",
  "gene_name": "D(3) dopamine receptor",
  "term_label": "phospholipase C-activating dopamine receptor signaling pathway",
  "gene": "UniProtKB:P35462"
}